{
  "gene": "UniProtKB:Q6R2W3",
  "term_id": "UNKNOWN:0003",
  "gene_symbol": "SCAND3",
  "term_label": "Unknown cellular component",
  "gene_name": "SCAN domain-containing protein 3"
}